{
  "gene": "UniProtKB:Q14997",
  "term_label": "peptidase activator activity",
  "gene_symbol": "PSME4",
  "gene_name": "Proteasome activator complex subunit 4",
  "term_id": "GO:0016504"
}